positive regulation of relaxation of cardiac muscle [GO:1901899] (biological process) References: PMID:19708671 Sources: GOC:BHF, GOC:TermGenie, GOC:rl Definition: Any process that activates or increases the frequency, rate or extent of relaxation of cardiac muscle. Also known as: up regulation of relaxation of cardiac muscle, up-regulation of relaxation of cardiac muscle, upregulation of relaxation of cardiac muscle, activation of relaxation of cardiac muscle Relationships: is a type of positive regulation of relaxation of muscle [GO:1901079]; is a type of regulation of relaxation of cardiac muscle [GO:1901897]; positively regulates GO:0055119